Kv4.2-KChIP4 channel complex [GO:0071195] (cellular component) Relationships: is_a voltage-gated potassium channel complex [GO:0008076] Definition: A voltage-gated potassium channel complex that contains the Kv channel interacting protein KChIP4 associated with the channel via interaction with the Kv alpha subunit 4.2. References: PMID:15356203